cellular response to light stimulus [GO:0071482] (biological process) Sources: GOC:mah Definition: Any process that results in a change in state or activity of a cell (in terms of movement, secretion, enzyme production, gene expression, etc.) as a result of a light stimulus, electromagnetic radiation of wavelengths classified as infrared, visible or ultraviolet light. Subtypes: G protein-coupled opsin signaling pathway [GO:0016056], cellular response to UV [GO:0034644], cellular response to blue light [GO:0071483], cellular response to light intensity [GO:0071484], GO:0071489 Relationships: is a type of response to light stimulus [GO:0009416]; is a type of cellular response to radiation [GO:0071478]